{
  "gene": "UniProtKB:P09237",
  "term_id": "GO:0030574",
  "term_label": "collagen catabolic process",
  "gene_symbol": "MMP7",
  "gene_name": "Matrilysin"
}